alpha-beta T cell proliferation involved in immune response [GO:0002310] (biological process) Definition: The expansion of an alpha-beta T cell population by cell division as part of an immune response. Also known as: alpha-beta T cell proliferation during immune response, alpha-beta T lymphocyte proliferation during immune response, alpha-beta T-cell proliferation during immune response, alpha-beta T-lymphocyte proliferation during immune response Relationships: is a type of alpha-beta T cell activation involved in immune response [GO:0002287]; is a type of T cell proliferation involved in immune response [GO:0002309]; is a type of GO:0046633 Subtypes: GO:0002289 Sources: GOC:add, ISBN:0781735149